{
  "term_id": "GO:0006357",
  "gene_symbol": "CRX",
  "gene": "UniProtKB:O43186",
  "gene_name": "Cone-rod homeobox protein",
  "term_label": "regulation of transcription by RNA polymerase II"
}